{
  "gene_name": "Regulator of G-protein signaling 8",
  "gene": "UniProtKB:P57771",
  "term_id": "GO:0005096",
  "term_label": "GTPase activator activity",
  "gene_symbol": "RGS8"
}